{
  "term_id": "GO:0007186",
  "gene_name": "Choriogonadotropin subunit beta 7",
  "term_label": "G protein-coupled receptor signaling pathway",
  "gene": "UniProtKB:P0DN87",
  "gene_symbol": "CGB7"
}